endonuclear canal [GO:0035843] (cellular component) References: PMID:18359585 Sources: GOC:bf Relationships: is a type of GO:0110165; BFO_0000050 GO:0001673 Definition: A membrane-bound structure present in the nucleus of a spermatozoon. There is variation in the number of endonuclear canals between sperm of different organisms, and some species lack these structures altogether. The endonuclear canal may provide a supporting role for the sperm nucleus, and originates during spermiogenesis from an invagination of the nuclear envelope.